{
  "term_id": "GO:0005654",
  "term_label": "nucleoplasm",
  "gene_symbol": "CDKN2AIP",
  "gene": "UniProtKB:Q9NXV6",
  "gene_name": "CDKN2A-interacting protein"
}